{
  "term_label": "glycolytic process",
  "gene_symbol": "GAPDH",
  "gene": "UniProtKB:P04406",
  "gene_name": "Glyceraldehyde-3-phosphate dehydrogenase",
  "term_id": "GO:0006096"
}